enterobactin transport [GO:0042930] (biological process) Definition: The directed movement of the siderochrome enterobactin, a cyclic trimer of 2, 3 dihydroxybenzoylserine into, out of or within a cell, or between cells, by means of some agent such as a transporter or pore. Relationships: is a type of organic anion transport [GO:0015711]; is a type of organic hydroxy compound transport [GO:0015850]; is_a siderophore transport [GO:0015891] Also known as: enterochelin transport Sources: GOC:jl